{
  "gene_name": "Protein lyl-1",
  "term_id": "GO:0000978",
  "term_label": "RNA polymerase II cis-regulatory region sequence-specific DNA binding",
  "gene_symbol": "LYL1",
  "gene": "UniProtKB:P12980"
}